{
  "term_id": "UNKNOWN:0003",
  "term_label": "Unknown cellular component",
  "gene": "UniProtKB:Q6ZVQ6",
  "gene_symbol": "Q6ZVQ6",
  "gene_name": "Putative uncharacterized protein FLJ42213"
}